{
  "gene_name": "Zinc finger protein 630",
  "gene_symbol": "ZNF630",
  "term_label": "DNA-binding transcription factor activity, RNA polymerase II-specific",
  "gene": "UniProtKB:Q2M218",
  "term_id": "GO:0000981"
}